{
  "gene_symbol": "KRT35",
  "gene_name": "Keratin, type I cuticular Ha5",
  "term_label": "intermediate filament organization",
  "gene": "UniProtKB:Q92764",
  "term_id": "GO:0045109"
}